{
  "term_id": "GO:0006613",
  "gene_symbol": "ARL6IP1",
  "term_label": "cotranslational protein targeting to membrane",
  "gene": "UniProtKB:Q15041",
  "gene_name": "ADP-ribosylation factor-like protein 6-interacting protein 1"
}